{
  "term_label": "histone binding",
  "gene_name": "Acidic leucine-rich nuclear phosphoprotein 32 family member E",
  "term_id": "GO:0042393",
  "gene_symbol": "ANP32E",
  "gene": "UniProtKB:Q9BTT0"
}